{
  "term_label": "signal transduction",
  "term_id": "GO:0007165",
  "gene_name": "Neurexin-3",
  "gene_symbol": "NRXN3",
  "gene": "UniProtKB:Q9Y4C0"
}